monodehydroascorbate reductase (NADH) activity [GO:0016656] (molecular function) Relationships: is a type of oxidoreductase activity, acting on NAD(P)H, quinone or similar compound as acceptor [GO:0016655] Definition: Catalysis of the reaction: 2 monodehydro-L-ascorbate radical + NADH + H+ = 2 L-ascorbate + NAD+. Also known as: monodehydroascorbate reductase activity, AFR, AFR-reductase activity, MDAsA reductase (NADPH), MDHA, NADH-semidehydroascorbate oxidoreductase activity, NADH:AFR oxidoreductase activity, NADH:ascorbate radical oxidoreductase activity, NADH:monodehydroascorbate oxidoreductase activity, NADH:semidehydroascorbic acid oxidoreductase activity, SDA reductase activity, ascorbate free radical reductase activity, ascorbate free-radical reductase activity, ascorbic free radical reductase activity, semidehydroascorbate reductase activity Sources: RHEA:14581